{
  "gene_name": "Putative makorin-5",
  "term_label": "Unknown biological process",
  "gene_symbol": "MKRN9P",
  "term_id": "UNKNOWN:0002",
  "gene": "UniProtKB:Q6NVV0"
}